{
  "gene": "UniProtKB:Q8WZ92",
  "gene_name": "Olfactory receptor 5P2",
  "term_label": "olfactory receptor activity",
  "gene_symbol": "OR5P2",
  "term_id": "GO:0004984"
}